{
  "term_id": "GO:0048066",
  "gene_symbol": "EDNRB",
  "term_label": "developmental pigmentation",
  "gene": "UniProtKB:P24530",
  "gene_name": "Endothelin receptor type B"
}